{
  "gene_symbol": "ADGRG6",
  "term_label": "adenylate cyclase-activating G protein-coupled receptor signaling pathway",
  "gene_name": "Adhesion G-protein coupled receptor G6",
  "gene": "UniProtKB:Q86SQ4",
  "term_id": "GO:0007189"
}